negative regulation of Roundabout signaling pathway [GO:0035387] (biological process) Definition: Any process that stops, prevents, or reduces the frequency, rate or extent of the Roundabout signaling pathway. Sources: GOC:BHF Also known as: negative regulation of Roundabout signalling pathway Relationships: is_a negative regulation of signal transduction [GO:0009968]; is a type of GO:0035386; RO_0002212 Roundabout signaling pathway [GO:0035385] Subtypes: termination of Roundabout signal transduction [GO:0035554]